{
  "term_id": "UNKNOWN:0002",
  "term_label": "Unknown biological process",
  "gene": "UniProtKB:Q7Z4B0",
  "gene_symbol": "LINC00305",
  "gene_name": "Putative uncharacterized protein encoded by LINC00305"
}